{
  "term_label": "protein-N-terminal-glutamate acetyltransferase activity",
  "gene": "UniProtKB:P41227",
  "term_id": "GO:1990190",
  "gene_name": "N-alpha-acetyltransferase 10",
  "gene_symbol": "NAA10"
}